{
  "term_label": "Unknown molecular function",
  "term_id": "UNKNOWN:0001",
  "gene_symbol": "ARMCX3",
  "gene": "UniProtKB:Q9UH62",
  "gene_name": "Armadillo repeat-containing X-linked protein 3"
}